{
  "term_id": "GO:0050840",
  "gene_symbol": "DMP1",
  "gene": "UniProtKB:Q13316",
  "term_label": "extracellular matrix binding",
  "gene_name": "Dentin matrix acidic phosphoprotein 1"
}